{
  "term_id": "GO:0004984",
  "gene": "UniProtKB:Q8NH06",
  "gene_symbol": "OR1P1",
  "term_label": "olfactory receptor activity",
  "gene_name": "Olfactory receptor 1P1"
}